{
  "term_label": "Unknown biological process",
  "gene_name": "EEF1A lysine methyltransferase 4",
  "gene": "UniProtKB:P0DPD7",
  "term_id": "UNKNOWN:0002",
  "gene_symbol": "EEF1AKMT4"
}